positive regulation of zygosporangium development [GO:0075273] (biological process) Definition: Any process that activates, maintains or increases the frequency, rate or extent of zygosporangium development, a process in which a fruiting body called zygosporangium is formed. Sources: GOC:pamgo_curators Relationships: is a type of GO:0075261; is a type of regulation of zygosporangium development [GO:0075272]; positively regulates zygosporangium development [GO:0075271]